{
  "term_label": "plasma membrane",
  "gene_symbol": "OR3A1",
  "gene": "UniProtKB:P47881",
  "term_id": "GO:0005886",
  "gene_name": "Olfactory receptor 3A1"
}